acetyl-CoA decarbonylase/synthase-carbon monoxide dehydrogenase complex [GO:0044672] (cellular component) Relationships: is a type of catalytic complex [GO:1902494] Also known as: CO dehydrogenase complex, CODH, carbon monoxide dehydrogenase, carbon-monoxide:(acceptor) oxidoreductase complex, CO dehydrogenase/acetyl-CoA synthase complex, CODH/ACS complex References: PMID:11607176, PMID:7693685, PMID:8955306 Sources: GOC:mengo_curators Definition: A multifunctional enzyme complex composed of five different polypeptides that catalyzes the decarbonylation of acetyl-CoA, cleaves the C-C and C-S bonds in the acetyl moiety of acetyl-CoA, oxidizes the carbonyl group to CO2 and transfers the methyl group to tetrahydrosarcinapterin. These reactions are important for methanogenesis.